{
  "term_label": "membrane",
  "gene": "UniProtKB:O75324",
  "gene_name": "Stannin",
  "term_id": "GO:0016020",
  "gene_symbol": "SNN"
}